{
  "gene_symbol": "FAU",
  "term_label": "cytosolic ribosome",
  "term_id": "GO:0022626",
  "gene_name": "Ubiquitin-like FUBI-ribosomal protein eS30 fusion protein",
  "gene": "UniProtKB:P62861"
}